{
  "gene_name": "Betaine--homocysteine S-methyltransferase 1",
  "term_label": "L-methionine salvage",
  "gene": "UniProtKB:Q93088",
  "term_id": "GO:0071267",
  "gene_symbol": "BHMT"
}